{
  "term_id": "GO:0038098",
  "term_label": "sequestering of BMP from receptor via BMP binding",
  "gene": "UniProtKB:P41271",
  "gene_name": "Neuroblastoma suppressor of tumorigenicity 1",
  "gene_symbol": "NBL1"
}